{
  "gene_name": "Kinesin-like protein KIF2C",
  "term_label": "cytoplasm",
  "gene": "UniProtKB:Q99661",
  "term_id": "GO:0005737",
  "gene_symbol": "KIF2C"
}